{
  "term_id": "GO:0006357",
  "gene_name": "E3 SUMO-protein ligase PIAS3",
  "gene_symbol": "PIAS3",
  "gene": "UniProtKB:Q9Y6X2",
  "term_label": "regulation of transcription by RNA polymerase II"
}